{
  "term_id": "GO:0000226",
  "gene_name": "Serine_threonine-protein kinase SIK3",
  "gene_symbol": "SIK3",
  "gene": "UniProtKB:Q9Y2K2",
  "term_label": "microtubule cytoskeleton organization"
}